protein localization to plasma membrane of cell tip [GO:1903418] (biological process) References: PMID:25157670, PMID:27852900 Sources: GOC:TermGenie, GO_REF:0000087 Also known as: protein localisation in plasma membrane of cell tip, protein localisation to plasma membrane of cell tip, protein localization in plasma membrane of cell tip Definition: A process in which a protein is transported to, or maintained in, a location within a plasma membrane of cell tip. Relationships: is a type of protein localization to membrane [GO:0072657]; is a type of GO:1990151; is a type of GO:1990778